{
  "gene": "UniProtKB:O15230",
  "gene_symbol": "LAMA5",
  "gene_name": "Laminin subunit alpha-5",
  "term_id": "GO:0005615",
  "term_label": "extracellular space"
}